{
  "gene": "UniProtKB:P22415",
  "term_id": "UNKNOWN:0003",
  "gene_name": "Upstream stimulatory factor 1",
  "term_label": "Unknown cellular component",
  "gene_symbol": "USF1"
}